complement binding [GO:0001848] (molecular function) Note: Note that the complement cascade includes all of the components involved in the classical complement pathway, the alternative complement pathway, and the lectin complement pathway, as well as the common components of all three pathways. Subtypes: complement component C1q complex binding [GO:0001849], complement component C3a binding [GO:0001850], complement component C3b binding [GO:0001851], complement component iC3b binding [GO:0001852], GO:0001853, GO:0001854, complement component C4b binding [GO:0001855], complement component C5a binding [GO:0001856] Sources: GOC:add, ISBN:0781735149 Definition: Binding to a component or product of the complement cascade. Relationships: is_a protein binding [GO:0005515]